{
  "gene": "UniProtKB:Q9NW07",
  "gene_name": "Zinc finger protein 358",
  "term_id": "UNKNOWN:0003",
  "gene_symbol": "ZNF358",
  "term_label": "Unknown cellular component"
}